{
  "gene_name": "Delta-like protein 3",
  "term_label": "plasma membrane",
  "gene": "UniProtKB:Q9NYJ7",
  "gene_symbol": "DLL3",
  "term_id": "GO:0005886"
}